{
  "gene_symbol": "ADSS1",
  "term_label": "cytoplasm",
  "gene_name": "Adenylosuccinate synthetase isozyme 1",
  "term_id": "GO:0005737",
  "gene": "UniProtKB:Q8N142"
}